opine dehydrogenase activity [GO:0047129] (MF) Relationships: is a type of oxidoreductase activity, acting on the CH-NH group of donors, NAD or NADP as acceptor [GO:0016646] Also known as: (2S)-2-{[1-(R)-carboxyethyl]amino}pentanoate dehydrogenase (NAD, L-aminopentanoate-forming), (2S)-2-{[1-(R)-carboxyethyl]amino}pentanoate:NAD+ oxidoreductase (L-aminopentanoate-forming) Definition: Catalysis of the reaction: (2S)-2-[(R)-1-carboxyethylamino]pentanoate + H2O + NAD+ = L-2-aminopentanoate + H+ + NADH + pyruvate. Sources: EC:1.5.1.28, RHEA:21592